negative regulation of trophoblast cell migration [GO:1901164] (biological process) Definition: Any process that stops, prevents or reduces the frequency, rate or extent of trophoblast cell migration. Sources: GOC:BHF, GOC:TermGenie Also known as: down regulation of trophoblast cell migration, down-regulation of trophoblast cell migration, downregulation of trophoblast cell migration, inhibition of trophoblast cell migration Relationships: is a type of negative regulation of cell migration [GO:0030336]; is a type of negative regulation of multicellular organismal process [GO:0051241]; is a type of GO:1901163; is a type of negative regulation of reproductive process [GO:2000242]; negatively regulates trophoblast cell migration [GO:0061450]